{
  "term_label": "L-malate dehydrogenase (NAD+) activity",
  "gene": "UniProtKB:Q5I0G3",
  "gene_symbol": "MDH1B",
  "gene_name": "Putative malate dehydrogenase 1B",
  "term_id": "GO:0030060"
}